{
  "gene_symbol": "ITPRIPL1",
  "gene": "UniProtKB:Q6GPH6",
  "gene_name": "Inositol 1,4,5-trisphosphate receptor-interacting protein-like 1",
  "term_id": "GO:0016020",
  "term_label": "membrane"
}